{
  "gene": "UniProtKB:O95631",
  "gene_name": "Netrin-1",
  "gene_symbol": "NTN1",
  "term_id": "GO:0006357",
  "term_label": "regulation of transcription by RNA polymerase II"
}